regulation of myosin II filament assembly [GO:0043520] (biological process) Sources: GOC:jl Relationships: is_a regulation of protein-containing complex assembly [GO:0043254]; is a type of regulation of myosin II filament organization [GO:0043519]; RO_0002211 myosin II filament assembly [GO:0031036] Subtypes: GO:1905510, positive regulation of myosin II filament assembly [GO:1905511] Definition: Any process that modulates the frequency, rate or extent of the formation of a bipolar filament composed of myosin II molecules.